{
  "term_id": "GO:0046928",
  "gene_symbol": "FER1L5",
  "term_label": "regulation of neurotransmitter secretion",
  "gene": "UniProtKB:A0AVI2",
  "gene_name": "Fer-1-like protein 5"
}